demethylkotanin catabolic process [GO:1900598] (BP) Sources: GOC:TermGenie, GOC:di Relationships: is_a secondary metabolite catabolic process [GO:0090487] Also known as: demethylkotanin breakdown, demethylkotanin catabolism, demethylkotanin degradation Definition: The chemical reactions and pathways resulting in the breakdown of demethylkotanin.